{
  "gene": "UniProtKB:Q9HCY8",
  "term_id": "GO:0005615",
  "gene_symbol": "S100A14",
  "gene_name": "Protein S100-A14",
  "term_label": "extracellular space"
}